adenosylmethionine decarboxylase activity [GO:0004014] (molecular function) Sources: EC:4.1.1.50, RHEA:15981 Definition: Catalysis of the reaction: S-adenosyl-L-methionine + H+ = S-adenosylmethioninamine + CO2. Also known as: adenosyl methionine decarboxylase activity, S-adenosyl-L-methionine carboxy-lyase [(5-deoxy-5-adenosyl)(3-aminopropyl)-methylsulfonium-salt-forming], S-adenosyl-L-methionine carboxy-lyase activity, S-adenosyl-L-methionine decarboxylase activity, S-adenosylmethionine decarboxylase activity Relationships: is_a carboxy-lyase activity [GO:0016831]